{
  "term_id": "GO:0051015",
  "gene_symbol": "ABLIM1",
  "gene": "UniProtKB:O14639",
  "gene_name": "Actin-binding LIM protein 1",
  "term_label": "actin filament binding"
}